{
  "term_label": "Unknown cellular component",
  "gene_symbol": "AKAP2",
  "gene": "UniProtKB:Q9Y2D5",
  "gene_name": "A-kinase anchor protein 2",
  "term_id": "UNKNOWN:0003"
}